{
  "term_label": "Unknown cellular component",
  "gene": "UniProtKB:Q9HCK4",
  "term_id": "UNKNOWN:0003",
  "gene_symbol": "ROBO2",
  "gene_name": "Roundabout homolog 2"
}